{
  "gene": "UniProtKB:Q9BUB5",
  "term_label": "calcium/calmodulin-dependent protein kinase activity",
  "gene_name": "MAP kinase-interacting serine_threonine-protein kinase 1",
  "term_id": "GO:0004683",
  "gene_symbol": "MKNK1"
}